pyrimidine nucleoside biosynthetic process [GO:0046134] (biological process) Relationships: is a type of GO:0006213; is a type of nucleoside biosynthetic process [GO:0009163]; is a type of pyrimidine-containing compound biosynthetic process [GO:0072528] Sources: GOC:ai Also known as: pyrimidine nucleoside anabolism, pyrimidine nucleoside biosynthesis, pyrimidine nucleoside formation, pyrimidine nucleoside synthesis Definition: The chemical reactions and pathways resulting in the formation of one of a family of organic molecules consisting of a pyrimidine base covalently bonded to a sugar ribose (a ribonucleoside) or deoxyribose (a deoxyribonucleoside). Subtypes: GO:0043097, pyrimidine deoxyribonucleoside biosynthetic process [GO:0046126], pyrimidine ribonucleoside biosynthetic process [GO:0046132], GO:1905266